protein localization to Mei2 nuclear dot [GO:1902549] (biological process) References: PMID:23980030 Sources: GOC:TermGenie Also known as: protein localisation in Mei2 nuclear dot, protein localisation to Mei2 nuclear dot, protein localization in Mei2 nuclear dot, protein localization to Mei2 dot Definition: A process in which a protein is transported to, or maintained in, a location within a Mei2 nuclear dot. Relationships: is a type of protein localization to nucleus [GO:0034504]